{
  "gene_name": "Programmed cell death protein 7",
  "gene": "UniProtKB:Q8N8D1",
  "term_label": "U12-type spliceosomal complex",
  "gene_symbol": "PDCD7",
  "term_id": "GO:0005689"
}